{
  "term_id": "GO:0015630",
  "term_label": "microtubule cytoskeleton",
  "gene_symbol": "SEPTIN2",
  "gene_name": "Septin-2",
  "gene": "UniProtKB:Q15019"
}